{
  "gene_name": "Poly [ADP-ribose] polymerase tankyrase-1",
  "gene_symbol": "TNKS",
  "term_id": "GO:1904355",
  "gene": "UniProtKB:O95271",
  "term_label": "positive regulation of telomere capping"
}